spindle checkpoint signaling [GO:0031577] (biological process) Note: Note that this term should not be used for direct manual annotation as it should always be possible to choose either a mitotic or meiotic child term. Also known as: signal transduction involved in spindle checkpoint, spindle checkpoint Relationships: is a type of GO:0000075 Sources: GOC:mtg_cell_cycle Subtypes: GO:0044779, GO:0071173, mitotic spindle checkpoint signaling [GO:0071174] Regulation: regulated by regulation of spindle checkpoint [GO:0090231]; positively regulated by positive regulation of spindle checkpoint [GO:0090232]; negatively regulated by negative regulation of spindle checkpoint [GO:0090233] Definition: A signaling process that that controls a cell cycle checkpoint that originates from the mitotic or meiotic spindle.